mRNA pseudouridine synthesis [GO:1990481] (biological process) Definition: The intramolecular conversion of uridine to pseudouridine in an mRNA molecule. Relationships: is a type of pseudouridine synthesis [GO:0001522]; is a type of GO:0016556 References: PMID:25192136 Also known as: mRNA pseudouridylation